rhombomere 2 development [GO:0021568] (biological process) Sources: GOC:cls, GOC:curators, GOC:dgh, GOC:dph, GOC:jid Definition: The process whose specific outcome is the progression of rhombomere 2 over time, from its formation to the mature structure. Rhombomeres are transverse segments of the developing rhombencephalon. Rhombomeres are lineage restricted, express different genes from one another, and adopt different developmental fates. Rhombomeres are numbered in anterior to posterior order. Relationships: is a type of rhombomere development [GO:0021546]